{
  "gene_name": "RNA polymerase II subunit A C-terminal domain phosphatase SSU72",
  "term_label": "termination of RNA polymerase II transcription",
  "gene": "UniProtKB:Q9NP77",
  "term_id": "GO:0006369",
  "gene_symbol": "SSU72"
}